{
  "gene_name": "Ig-like domain-containing protein (Fragment)",
  "gene": "UniProtKB:A0A087WW49",
  "gene_symbol": "LOC102724971",
  "term_id": "GO:0003823",
  "term_label": "antigen binding"
}